{
  "gene_name": "5'-nucleotidase domain-containing protein 2",
  "term_id": "UNKNOWN:0002",
  "gene_symbol": "NT5DC2",
  "term_label": "Unknown biological process",
  "gene": "UniProtKB:Q9H857"
}